{
  "term_id": "UNKNOWN:0001",
  "gene": "UniProtKB:Q96G27",
  "gene_name": "WW domain-binding protein 1",
  "term_label": "Unknown molecular function",
  "gene_symbol": "WBP1"
}